caveola neck [GO:0099400] (cellular component) References: PMID:17227843 Sources: GOC:PARL, GOC:pad Relationships: is a type of plasma membrane region [GO:0098590]; is a type of membrane microdomain [GO:0098857]; is part of GO:0005901 Definition: A membrane microdomain that forms a necklace around the bulb (crater) of a caveola. Intramembrane particles are concentrated in this region and cytoskeletal components, including actin, are highly enriched in the area underlying it.